{
  "term_label": "innate immune response",
  "gene": "UniProtKB:Q14142",
  "gene_name": "Tripartite motif-containing protein 14",
  "term_id": "GO:0045087",
  "gene_symbol": "TRIM14"
}